{
  "term_id": "UNKNOWN:0002",
  "gene": "UniProtKB:Q8NBZ9",
  "gene_symbol": "NEXN-AS1",
  "gene_name": "Putative uncharacterized protein NEXN-AS1",
  "term_label": "Unknown biological process"
}